{
  "term_label": "Unknown molecular function",
  "gene": "UniProtKB:A0A1B0GUA9",
  "gene_symbol": "C13orf46",
  "gene_name": "Uncharacterized protein C13orf46",
  "term_id": "UNKNOWN:0001"
}